response to mycotoxin [GO:0010046] (biological process) Definition: Any process that results in a change in state or activity of a cell or an organism (in terms of movement, secretion, enzyme production, gene expression, etc.) as a result of a mycotoxin stimulus. A mycotoxin is a toxic chemical substance produced by fungi. Sources: GOC:sm Relationships: is a type of GO:0009636 Subtypes: cellular response to mycotoxin [GO:0036146]